{
  "term_label": "double-stranded DNA 3'-5' DNA exonuclease activity",
  "term_id": "GO:0008311",
  "gene_name": "DNA-(apurinic or apyrimidinic site) endonuclease",
  "gene": "UniProtKB:P27695",
  "gene_symbol": "APEX1"
}